MHC class II protein binding, via lateral surface [GO:0042657] (molecular function) Relationships: is a type of MHC class II protein binding [GO:0042289] Also known as: major histocompatibility complex class II protein binding, via lateral surface Definition: Binding to the lateral surface of major histocompatibility complex class II molecules. Sources: GOC:jl